response to palmitoleic acid [GO:1904926] (biological process) Relationships: is a type of GO:0070542 References: PMID:25429233 Sources: GOC:TermGenie, GOC:mr, GO_REF:0000071 Definition: Any process that results in a change in state or activity of a cell or an organism (in terms of movement, secretion, enzyme production, gene expression, etc.) as a result of a palmitoleic acid stimulus. Subtypes: cellular response to palmitoleic acid [GO:1904927]